{
  "term_id": "GO:0030018",
  "gene_name": "PDZ and LIM domain protein 5",
  "gene": "UniProtKB:Q96HC4",
  "gene_symbol": "PDLIM5",
  "term_label": "Z disc"
}